{
  "gene_name": "ATP synthase membrane subunit K, mitochondrial",
  "term_id": "UNKNOWN:0002",
  "term_label": "Unknown biological process",
  "gene_symbol": "ATP5MK",
  "gene": "UniProtKB:Q96IX5"
}